{
  "gene_symbol": "PHLPP2",
  "term_id": "UNKNOWN:0001",
  "gene": "UniProtKB:Q6ZVD8",
  "gene_name": "PH domain leucine-rich repeat-containing protein phosphatase 2",
  "term_label": "Unknown molecular function"
}